{
  "term_id": "GO:0005634",
  "gene_symbol": "ZNF784",
  "term_label": "nucleus",
  "gene_name": "Zinc finger protein 784",
  "gene": "UniProtKB:Q8NCA9"
}